{
  "term_id": "UNKNOWN:0001",
  "gene_name": "Small EDRK-rich factor 2",
  "gene": "UniProtKB:P84101",
  "gene_symbol": "SERF2",
  "term_label": "Unknown molecular function"
}